{
  "gene_name": "Proto-oncogene Wnt-1",
  "term_label": "canonical Wnt signaling pathway",
  "gene": "UniProtKB:P04628",
  "term_id": "GO:0060070",
  "gene_symbol": "WNT1"
}